exoxylanase activity [GO:0097600] (molecular function) Definition: A xylanase activity that acts on one of the ends of a xylan polymer which does not contain side chains. References: PMID:16535010 Sources: GOC:jh2, ISBN:81-7736-269-0 Relationships: is_a GO:0097599